{
  "gene_symbol": "ARFGEF1",
  "gene_name": "Brefeldin A-inhibited guanine nucleotide-exchange protein 1",
  "gene": "UniProtKB:Q9Y6D6",
  "term_id": "GO:0007030",
  "term_label": "Golgi organization"
}